{
  "gene_symbol": "LMAN1L",
  "term_label": "D-mannose binding",
  "term_id": "GO:0005537",
  "gene": "UniProtKB:Q9HAT1",
  "gene_name": "Protein ERGIC-53-like"
}